{
  "gene_name": "Gamma-aminobutyric acid receptor-associated protein-like 3",
  "term_id": "GO:0031625",
  "gene_symbol": "GABARAPL3",
  "gene": "UniProtKB:Q9BY60",
  "term_label": "ubiquitin protein ligase binding"
}